{
  "term_label": "DNA binding",
  "gene": "UniProtKB:Q99879",
  "term_id": "GO:0003677",
  "gene_symbol": "H2BC14",
  "gene_name": "Histone H2B type 1-M"
}